{
  "gene_name": "Ras-specific guanine nucleotide-releasing factor RalGPS1",
  "gene": "UniProtKB:Q5JS13",
  "term_label": "regulation of Ral protein signal transduction",
  "term_id": "GO:0032485",
  "gene_symbol": "RALGPS1"
}